{
  "gene_symbol": "PKD2",
  "gene_name": "Polycystin-2",
  "gene": "UniProtKB:Q13563",
  "term_id": "GO:0005102",
  "term_label": "signaling receptor binding"
}